{
  "term_id": "GO:0005543",
  "gene_name": "Pleckstrin homology domain-containing family A member 1",
  "gene_symbol": "PLEKHA1",
  "gene": "UniProtKB:Q9HB21",
  "term_label": "phospholipid binding"
}